detection of pH by chemoreceptor signaling [GO:0003022] (biological process) Relationships: is a type of detection of hydrogen ion [GO:0003030] Definition: The process in which information about the levels of hydrogen ions are received and are converted to a molecular signal by chemoreceptors. Also known as: detection of pH by chemoreceptor signalling Sources: GOC:mtg_cardio, ISBN:0323031951 Subtypes: detection of pH by aortic body chemoreceptor signaling [GO:0003036], GO:0003037